{
  "term_id": "GO:0030175",
  "gene_symbol": "GPM6A",
  "term_label": "filopodium",
  "gene": "UniProtKB:P51674",
  "gene_name": "Neuronal membrane glycoprotein M6-a"
}